{
  "gene_name": "snRNA-activating protein complex subunit 1",
  "term_label": "snRNA-activating protein complex",
  "gene": "UniProtKB:Q16533",
  "gene_symbol": "SNAPC1",
  "term_id": "GO:0019185"
}